{
  "gene_symbol": "TRAF1",
  "gene_name": "TNF receptor-associated factor 1",
  "term_id": "GO:0033209",
  "gene": "UniProtKB:Q13077",
  "term_label": "tumor necrosis factor-mediated signaling pathway"
}